posterior cibarial plate development [GO:0048727] (biological process) Sources: GOC:rc Definition: The process whose specific outcome is the progression of the posterior cibarial plate over time, from its formation to the mature structure. Relationships: is a type of anatomical structure development [GO:0048856]; is part of GO:0035213